{
  "term_label": "RNA polymerase II cis-regulatory region sequence-specific DNA binding",
  "gene_symbol": "ZNF141",
  "term_id": "GO:0000978",
  "gene": "UniProtKB:Q15928",
  "gene_name": "Zinc finger protein 141"
}